{
  "term_label": "nucleus",
  "gene_name": "NFIL3 like protein",
  "term_id": "GO:0005634",
  "gene": "UniProtKB:A0A5F9ZHS7",
  "gene_symbol": "NFILZ"
}